{
  "gene": "UniProtKB:Q14534",
  "term_id": "GO:0004506",
  "gene_name": "Squalene monooxygenase",
  "gene_symbol": "SQLE",
  "term_label": "squalene monooxygenase activity"
}